hyaluronan biosynthetic process [GO:0030213] (biological process) Regulation: regulated by GO:1900125; negatively regulated by negative regulation of hyaluronan biosynthetic process [GO:1900126]; positively regulated by positive regulation of hyaluronan biosynthetic process [GO:1900127] Definition: The chemical reactions and pathways resulting in the formation of hyaluronan, the naturally occurring anionic form of hyaluronic acid. Hyaluronan is a type of non-sulfated glycosaminoglycan composed of the repeating disaccharide unit beta(1,4)-D-glucuronic acid-beta(1,3)-N-acetyl-D-glucosamine. References: PMID:33171800, PMID:35536932 Relationships: is a type of glycosaminoglycan biosynthetic process [GO:0006024]; is a type of hyaluronan metabolic process [GO:0030212] Also known as: hyaluronan anabolism, hyaluronan biosynthesis, hyaluronan formation, hyaluronan synthesis